{
  "gene_name": "V-set and immunoglobulin domain-containing protein 10-like",
  "term_id": "UNKNOWN:0002",
  "gene_symbol": "VSIG10L",
  "term_label": "Unknown biological process",
  "gene": "UniProtKB:Q86VR7"
}